{
  "term_label": "protein kinase A regulatory subunit binding",
  "gene_symbol": "PRRC1",
  "term_id": "GO:0034237",
  "gene": "UniProtKB:Q96M27",
  "gene_name": "Protein PRRC1"
}